{
  "gene_symbol": "UBXN2A",
  "gene_name": "UBX domain-containing protein 2A",
  "term_label": "Golgi organization",
  "gene": "UniProtKB:P68543",
  "term_id": "GO:0007030"
}